{
  "term_id": "GO:0050694",
  "gene_name": "Galactose-3-O-sulfotransferase 3",
  "gene_symbol": "GAL3ST3",
  "gene": "UniProtKB:Q96A11",
  "term_label": "galactose 3-O-sulfotransferase activity"
}